{
  "gene_symbol": "BTBD16",
  "gene_name": "BTB_POZ domain-containing protein 16",
  "term_id": "UNKNOWN:0002",
  "term_label": "Unknown biological process",
  "gene": "UniProtKB:Q32M84"
}